(S)-cheilanthifoline synthase activity [GO:0047053] (molecular function) Sources: RHEA:20485 Also known as: (S)-scoulerine oxidase (methylenedioxy-bridge-forming) activity Definition: Catalysis of the reaction: (S)-scoulerine + [reduced NADPH--hemoprotein reductase] + O2 = (S)-cheilanthifoline + [oxidized NADPH--hemoprotein reductase] + 2 H2O. Relationships: is a type of GO:0016717